{
  "gene_symbol": "MTX3",
  "term_id": "GO:0001401",
  "gene": "UniProtKB:Q5HYI7",
  "term_label": "SAM complex",
  "gene_name": "Metaxin-3"
}